{
  "gene_symbol": "NSD3",
  "gene_name": "Histone-lysine N-methyltransferase NSD3",
  "term_id": "GO:0046975",
  "gene": "UniProtKB:Q9BZ95",
  "term_label": "histone H3K36 methyltransferase activity"
}